{
  "gene_name": "Olfactomedin-4",
  "term_id": "UNKNOWN:0001",
  "term_label": "Unknown molecular function",
  "gene_symbol": "OLFM4",
  "gene": "UniProtKB:Q6UX06"
}